{
  "term_id": "GO:0043065",
  "gene_name": "TCF3 fusion partner",
  "term_label": "positive regulation of apoptotic process",
  "gene": "UniProtKB:P0C1Z6",
  "gene_symbol": "TFPT"
}